{
  "term_id": "GO:0005737",
  "gene": "UniProtKB:Q9UJW3",
  "term_label": "cytoplasm",
  "gene_name": "DNA (cytosine-5)-methyltransferase 3-like",
  "gene_symbol": "DNMT3L"
}